typhasterol C-23 hydroxylase activity [GO:0102733] (molecular function) References: PMID:17138693 Sources: GOC:pz Relationships: is_a monooxygenase activity [GO:0004497]; is a type of oxidoreductase activity, acting on paired donors, with incorporation or reduction of molecular oxygen [GO:0016705] Definition: Catalysis of the reaction: typhasterol + O2 + a reduced electron acceptor = castasterone + H2O + an oxidized electron acceptor.